inositol-1,5-bisdiphosphate-2,3,4,6-tetrakisphosphate 1-diphosphatase activity [GO:0052846] (molecular function) References: PMID:10827188, PMID:11502751, PMID:26422458 Definition: Catalysis of the reaction: 1,5-bisdiphospho-1D-myo-inositol 2,3,4,6-tetrakisphosphate + H2O = 5-diphospho-1D-myo-inositol 1,2,3,4,6-pentakisphosphate + phosphate + H+. Relationships: is a type of inositol bisdiphosphate tetrakisphosphate diphosphatase activity [GO:0052841] Also known as: inositol 1,5-bisdiphosphate 2,3,4,6-tetrakisphosphate 1-diphosphatase activity, inositol 1,5-bispyrophosphate 2,3,4,6-tetrakisphosphate 1-pyrophosphatase activity